{
  "gene_name": "DnaJ homolog subfamily B member 14",
  "term_label": "Hsp70 protein binding",
  "gene": "UniProtKB:Q8TBM8",
  "term_id": "GO:0030544",
  "gene_symbol": "DNAJB14"
}